ribose-5-phosphate-ammonia ligase activity [GO:0050260] (molecular function) Relationships: is a type of GO:0016879 Also known as: 5-phosphoribosylamine synthetase activity, ammonia-ribose 5-phosphate aminotransferase activity, ribose 5-phosphate aminotransferase activity, ribose-5-phosphate:ammonia ligase (ADP-forming) Sources: EC:6.3.4.7, RHEA:13777 Definition: Catalysis of the reaction: D-ribose 5-phosphate + ATP + NH4 = 5-phospho-D-ribosylamine + ADP + 2 H+ + phosphate.